{
  "gene_name": "Microtubule nucleation factor SSNA1",
  "term_id": "GO:0005813",
  "term_label": "centrosome",
  "gene": "UniProtKB:O43805",
  "gene_symbol": "SSNA1"
}